Ras palmitoyltransferase activity [GO:0043849] (molecular function) References: PMID:16000296 Relationships: is a type of GO:0019706 Also known as: Ras protein acyltransferase activity, DHHC cysteine-rich domain-containing protein ERF2, ERF2, palmitoyltransferase ERF2 Definition: Catalysis of the reaction: palmitoyl-CoA + protein-cysteine = S-palmitoyl protein + CoA, specific for Ras proteins.